primary amino compound biosynthetic process [GO:1901162] (biological process) Relationships: is a type of biosynthetic process [GO:0009058] Subtypes: serotonin biosynthetic process [GO:0042427], phenylethylamine biosynthetic process [GO:0042444], chrysobactin biosynthetic process [GO:0042858], GO:0046335, agmatine biosynthetic process [GO:0097055], tyramine biosynthetic process [GO:1901695] Definition: The chemical reactions and pathways resulting in the formation of primary amino compound. Also known as: primary amino compound anabolism, primary amino compound biosynthesis, primary amino compound formation, primary amino compound synthesis Sources: GOC:TermGenie